{
  "gene_symbol": "MBOAT7",
  "term_id": "GO:0006661",
  "term_label": "phosphatidylinositol biosynthetic process",
  "gene_name": "Lysophospholipid acyltransferase 7",
  "gene": "UniProtKB:Q96N66"
}